{
  "term_id": "GO:0006436",
  "gene_symbol": "WARS1",
  "term_label": "tryptophanyl-tRNA aminoacylation",
  "gene": "UniProtKB:P23381",
  "gene_name": "Tryptophan--tRNA ligase, cytoplasmic"
}